{
  "term_label": "cyclin-dependent protein serine/threonine kinase regulator activity",
  "gene_name": "G1_S-specific cyclin-D2",
  "gene_symbol": "CCND2",
  "term_id": "GO:0016538",
  "gene": "UniProtKB:P30279"
}